{
  "gene": "UniProtKB:Q9Y2C3",
  "term_id": "GO:0008499",
  "gene_symbol": "B3GALT5",
  "term_label": "N-acetyl-beta-D-glucosaminide beta-(1,3)-galactosyltransferase activity",
  "gene_name": "Beta-1,3-galactosyltransferase 5"
}